gene conversion [GO:0035822] (biological process) References: PMID:17846636 Sources: GOC:mah Definition: A DNA recombination process that results in the unidirectional transfer of genetic material from a donor sequence to a highly homologous acceptor. The resulting acceptor sequence is identical to that of the donor. Relationships: is a type of homologous recombination [GO:0035825] Subtypes: gene conversion of immunoglobulin genes [GO:0002206], meiotic gene conversion [GO:0006311], gene conversion at mating-type locus [GO:0007534], GO:0035823, long tract gene conversion [GO:0035824]